{
  "gene_symbol": "TFIP11",
  "gene": "UniProtKB:Q9UBB9",
  "term_label": "U2-type post-mRNA release spliceosomal complex",
  "gene_name": "Tuftelin-interacting protein 11",
  "term_id": "GO:0071008"
}